lung neuroendocrine cell differentiation [GO:0061100] (biological process) Definition: The process in which a relatively unspecialized cell acquires specialized features of a neuroendocrine cell of the lung epithelium. References: PMID:9126746 Sources: GOC:dph Relationships: is a type of neuroendocrine cell differentiation [GO:0061101]; is a type of GO:0061140